{
  "gene_name": "Coiled-coil domain-containing protein 3",
  "gene": "UniProtKB:Q9BQI4",
  "term_label": "Unknown molecular function",
  "gene_symbol": "CCDC3",
  "term_id": "UNKNOWN:0001"
}